{
  "gene": "UniProtKB:Q8N131",
  "gene_name": "Porimin",
  "term_id": "UNKNOWN:0002",
  "term_label": "Unknown biological process",
  "gene_symbol": "TMEM123"
}